{
  "gene_symbol": "GOLIM4",
  "term_id": "GO:0005794",
  "gene": "UniProtKB:O00461",
  "term_label": "Golgi apparatus",
  "gene_name": "Golgi integral membrane protein 4"
}